{
  "gene": "UniProtKB:Q52LG2",
  "gene_name": "Keratin-associated protein 13-2",
  "term_id": "UNKNOWN:0003",
  "term_label": "Unknown cellular component",
  "gene_symbol": "KRTAP13-2"
}